{
  "term_id": "GO:0032020",
  "gene_name": "Ubiquitin-like protein ISG15",
  "term_label": "ISG15-protein conjugation",
  "gene_symbol": "ISG15",
  "gene": "UniProtKB:P05161"
}